{
  "gene_symbol": "XPR1",
  "term_id": "GO:0000822",
  "gene_name": "Solute carrier family 53 member 1",
  "term_label": "inositol hexakisphosphate binding",
  "gene": "UniProtKB:Q9UBH6"
}